{
  "gene": "UniProtKB:O00141",
  "gene_name": "Serine_threonine-protein kinase Sgk1",
  "gene_symbol": "SGK1",
  "term_label": "nucleus",
  "term_id": "GO:0005634"
}